{
  "term_label": "SCF ubiquitin ligase complex",
  "gene_symbol": "FBXL13",
  "gene_name": "F-box and leucine-rich repeat protein 13",
  "term_id": "GO:0019005",
  "gene": "UniProtKB:Q8NEE6"
}